{
  "term_label": "TFIIIC-class transcription factor complex binding",
  "gene": "UniProtKB:A6H8Y1",
  "gene_name": "Transcription factor TFIIIB component B'' homolog",
  "gene_symbol": "BDP1",
  "term_id": "GO:0001156"
}